bacteriochlorophyll binding [GO:0042314] (molecular function) Definition: Binding to bacteriochlorophyll, a form of chlorophyll found in photosynthetic bacteria, such as the purple and green bacteria. There are several types, designated a to g. Bacteriochlorophyll a and bacteriochlorophyll b are structurally similar to the chlorophyll a and chlorophyll b found in plants. Sources: ISBN:0192800981 Relationships: is a type of GO:0016168 Subtypes: bacteriochlorophyll c binding [GO:0016169]